{
  "gene_name": "Leukocyte receptor cluster member 1",
  "term_label": "Unknown biological process",
  "gene_symbol": "LENG1",
  "term_id": "UNKNOWN:0002",
  "gene": "UniProtKB:Q96BZ8"
}